{
  "gene_name": "Transmembrane emp24 domain-containing protein 2",
  "gene_symbol": "TMED2",
  "gene": "UniProtKB:Q15363",
  "term_id": "GO:0030134",
  "term_label": "COPII-coated ER to Golgi transport vesicle"
}